{
  "term_label": "guanylate cyclase complex, soluble",
  "gene_name": "Guanylate cyclase soluble subunit alpha-1",
  "term_id": "GO:0008074",
  "gene": "UniProtKB:Q02108",
  "gene_symbol": "GUCY1A1"
}